{
  "gene_symbol": "PCK2",
  "term_label": "response to starvation",
  "gene_name": "Phosphoenolpyruvate carboxykinase [GTP], mitochondrial",
  "term_id": "GO:0042594",
  "gene": "UniProtKB:Q16822"
}